mitochondrion [GO:0005739] (cellular component) Note: Some anaerobic or microaerophilic organisms (e.g. Entamoeba histolytica, Giardia intestinalis and several Microsporidia species) do not have mitochondria, and contain mitochondrion-related organelles (MROs) instead, called mitosomes or hydrogenosomes, very likely derived from mitochondria. To annotate gene products located in these mitochondrial relics in species such as Entamoeba histolytica, Giardia intestinalis or others, please use GO:0032047 'mitosome' or GO:0042566 'hydrogenosome'. (See PMID:24316280 for a list of species currently known to contain mitochondrion-related organelles.) Also known as: mitochondria Relationships: is a type of intracellular membrane-bounded organelle [GO:0043231]; is part of cytoplasm [GO:0005737] Sources: GOC:giardia, ISBN:0198506732 Definition: A semiautonomous, self replicating organelle that occurs in varying numbers, shapes, and sizes in the cytoplasm of virtually all eukaryotic cells. It is notably the site of tissue respiration.